{
  "gene": "UniProtKB:P0C7I0",
  "term_id": "GO:0005829",
  "term_label": "cytosol",
  "gene_name": "Inactive ubiquitin carboxyl-terminal hydrolase 17-like protein 8",
  "gene_symbol": "USP17L8"
}